{
  "gene_name": "Intersectin-1",
  "term_id": "GO:0097708",
  "term_label": "intracellular vesicle",
  "gene": "UniProtKB:Q15811",
  "gene_symbol": "ITSN1"
}